{
  "gene_symbol": "TLR7",
  "term_label": "canonical NF-kappaB signal transduction",
  "gene": "UniProtKB:Q9NYK1",
  "gene_name": "Toll-like receptor 7",
  "term_id": "GO:0007249"
}